{
  "gene_name": "Putative uncharacterized protein UNQ6494_PRO21346",
  "gene": "UniProtKB:Q6UXR6",
  "term_id": "UNKNOWN:0002",
  "term_label": "Unknown biological process",
  "gene_symbol": "UNQ6494_PRO21346"
}